{
  "term_id": "UNKNOWN:0003",
  "gene": "UniProtKB:Q5JRV8",
  "gene_name": "Transmembrane protein 255A",
  "gene_symbol": "TMEM255A",
  "term_label": "Unknown cellular component"
}